pyrimidine ribonucleoside monophosphate biosynthetic process [GO:0009174] (biological process) Also known as: pyrimidine ribonucleoside monophosphate anabolism, pyrimidine ribonucleoside monophosphate biosynthesis, pyrimidine ribonucleoside monophosphate formation, pyrimidine ribonucleoside monophosphate synthesis Definition: The chemical reactions and pathways resulting in the formation of pyrimidine ribonucleoside monophosphate, a compound consisting of a pyrimidine base linked to a ribose sugar esterified with phosphate on the sugar. Sources: GOC:go_curators, ISBN:0198506732 Subtypes: UMP biosynthetic process [GO:0006222], GO:0006230, GO:0009224 Relationships: is a type of pyrimidine nucleoside monophosphate biosynthetic process [GO:0009130]; is a type of ribonucleoside monophosphate biosynthetic process [GO:0009156]; is a type of pyrimidine ribonucleoside monophosphate metabolic process [GO:0009173]